{
  "gene": "UniProtKB:Q1L5Z9",
  "gene_name": "LON peptidase N-terminal domain and RING finger protein 2",
  "term_id": "GO:0061630",
  "term_label": "ubiquitin protein ligase activity",
  "gene_symbol": "LONRF2"
}